{
  "term_label": "extracellular space",
  "gene_symbol": "CUZD1",
  "gene_name": "CUB and zona pellucida-like domain-containing protein 1",
  "gene": "UniProtKB:Q86UP6",
  "term_id": "GO:0005615"
}